{
  "gene": "UniProtKB:Q96L73",
  "gene_symbol": "NSD1",
  "term_id": "GO:0005634",
  "gene_name": "Histone-lysine N-methyltransferase, H3 lysine-36 specific",
  "term_label": "nucleus"
}